UDP-D-apiose synthase activity [GO:0102765] (molecular function) Sources: RHEA:70523 Relationships: is a type of carboxy-lyase activity [GO:0016831] Definition: Catalysis of the reaction: UDP-alpha-D-glucuronate + H+ = UDP-alpha-D-apiose + CO2.